regulation of circadian sleep/wake cycle [GO:0042749] (biological process) Sources: GOC:jl Subtypes: GO:0010840, GO:0045187 Definition: Any process that modulates the frequency, rate or extent of the circadian sleep/wake cycle. Relationships: is a type of regulation of circadian rhythm [GO:0042752]; is a type of GO:0050795; regulates circadian sleep/wake cycle [GO:0042745]